{
  "gene_name": "Protein unc-119 homolog B",
  "gene_symbol": "UNC119B",
  "gene": "UniProtKB:A6NIH7",
  "term_id": "GO:0060271",
  "term_label": "cilium assembly"
}